positive regulation of cardiac muscle cell proliferation [GO:0060045] (biological process) Relationships: is a type of positive regulation of cell population proliferation [GO:0008284]; is_a positive regulation of cardiac muscle tissue growth [GO:0055023]; is a type of regulation of cardiac muscle cell proliferation [GO:0060043]; positively regulates cardiac muscle cell proliferation [GO:0060038] Also known as: positive regulation of heart muscle cell proliferation Sources: GOC:dph, GOC:rph Definition: Any process that activates or increases the frequency, rate or extent of cardiac muscle cell proliferation.